monoamine:proton antiporter activity [GO:0015311] (MF) Relationships: is a type of GO:0008504; is a type of proton transmembrane transporter activity [GO:0015078]; is a type of antiporter activity [GO:0015297] Sources: TC:2.A.1.2.11, TC:2.A.1.2.12 Also known as: monoamine:hydrogen antiporter activity Definition: Enables the transfer of a solute or solutes from one side of a membrane to the other according to the reaction: H+(out) + monoamine(in) = H+(in) + monoamine(out).